{
  "term_id": "UNKNOWN:0003",
  "gene": "UniProtKB:Q9NV23",
  "gene_symbol": "OLAH",
  "term_label": "Unknown cellular component",
  "gene_name": "S-acyl fatty acid synthase thioesterase, medium chain"
}